{
  "gene_name": "ETS domain-containing protein Elk-3",
  "gene": "UniProtKB:P41970",
  "term_id": "GO:0030154",
  "gene_symbol": "ELK3",
  "term_label": "cell differentiation"
}